{
  "gene_name": "G protein-regulated inducer of neurite outgrowth 2",
  "gene": "UniProtKB:O60269",
  "term_label": "neuron projection development",
  "term_id": "GO:0031175",
  "gene_symbol": "GPRIN2"
}